{
  "gene_symbol": "S100A16",
  "gene": "UniProtKB:Q96FQ6",
  "term_label": "calcium ion binding",
  "term_id": "GO:0005509",
  "gene_name": "Protein S100-A16"
}